{
  "term_label": "DNA-binding transcription factor activity, RNA polymerase II-specific",
  "term_id": "GO:0000981",
  "gene": "UniProtKB:Q6AHZ1",
  "gene_name": "Zinc finger protein 518A",
  "gene_symbol": "ZNF518A"
}